{
  "term_label": "calcium ion binding",
  "gene": "UniProtKB:O75838",
  "gene_symbol": "CIB2",
  "term_id": "GO:0005509",
  "gene_name": "Calcium and integrin-binding family member 2"
}